{
  "gene_symbol": "SLC14A2",
  "gene": "UniProtKB:Q15849",
  "term_label": "urea transmembrane transport",
  "term_id": "GO:0071918",
  "gene_name": "Urea transporter 2"
}